oxidoreductase activity, acting on the CH-OH group of donors, cytochrome as acceptor [GO:0016898] (molecular function) Subtypes: D-lactate dehydrogenase (cytochrome) activity [GO:0004458], L-lactate dehydrogenase (cytochrome) activity [GO:0004460], D-lactate dehydrogenase (cytochrome c-553) activity [GO:0047051], polyvinyl alcohol dehydrogenase (cytochrome) activity [GO:0047059], mannitol dehydrogenase (cytochrome) activity [GO:0050087], alcohol dehydrogenase (cytochrome c(L)) activity [GO:0052933], alcohol dehydrogenase (cytochrome c) activity [GO:0052934] Sources: GOC:ai Definition: Catalysis of an oxidation-reduction (redox) reaction in which a CH-OH group acts as a hydrogen or electron donor and reduces a cytochrome molecule. Relationships: is a type of oxidoreductase activity, acting on CH-OH group of donors [GO:0016614]